{
  "gene": "UniProtKB:Q96Q89",
  "gene_symbol": "KIF20B",
  "gene_name": "Kinesin-like protein KIF20B",
  "term_id": "GO:0005874",
  "term_label": "microtubule"
}